{
  "gene": "UniProtKB:Q15361",
  "gene_name": "Transcription termination factor 1",
  "term_label": "nucleolus",
  "term_id": "GO:0005730",
  "gene_symbol": "TTF1"
}